{
  "term_label": "positive regulation of blood pressure",
  "term_id": "GO:0045777",
  "gene_name": "Tachykinin-3",
  "gene": "UniProtKB:Q9UHF0",
  "gene_symbol": "TAC3"
}